negative regulation of oocyte maturation [GO:1900194] (biological process) Subtypes: negative regulation of meiotic cell cycle process involved in oocyte maturation [GO:1904145] Also known as: down regulation of oocyte maturation, down-regulation of oocyte maturation, downregulation of oocyte maturation, inhibition of oocyte maturation Definition: Any process that stops, prevents or reduces the frequency, rate or extent of oocyte maturation. Relationships: is a type of GO:1900193; is a type of GO:1903430; is_a negative regulation of reproductive process [GO:2000242]; negatively regulates GO:0001556 Sources: GOC:TermGenie, GOC:kmv